{
  "gene": "UniProtKB:Q8TBC4",
  "term_label": "NEDD8 activating enzyme activity",
  "gene_symbol": "UBA3",
  "gene_name": "NEDD8-activating enzyme E1 catalytic subunit",
  "term_id": "GO:0019781"
}